{
  "gene": "UniProtKB:P28068",
  "term_label": "MHC class II protein complex binding",
  "gene_name": "HLA class II histocompatibility antigen, DM beta chain",
  "gene_symbol": "HLA-DMB",
  "term_id": "GO:0023026"
}